mitotic centrosome separation [GO:0007100] (biological process) Relationships: is a type of centrosome separation [GO:0051299]; is a type of GO:1903047; is part of GO:0140014 Definition: Separation of duplicated centrosome components at the beginning of mitosis. The centriole pair within each centrosome becomes part of a separate microtubule organizing center that nucleates a radial array of microtubules called an aster. The two asters move to opposite sides of the nucleus to form the two poles of the mitotic spindle. Regulation: regulated by regulation of mitotic centrosome separation [GO:0046602]; negatively regulated by negative regulation of mitotic centrosome separation [GO:0046603]; positively regulated by positive regulation of mitotic centrosome separation [GO:0046604] Sources: ISBN:0815316194